visceral serous pericardium development [GO:0061032] (biological process) Definition: The progression of the visceral serous pericardium from its formation to the mature structure. The visceral serous pericardium is the inner layer of the pericardium. Sources: GOC:dph, GOC:yaf Also known as: epicardium development Relationships: is a type of anatomical structure development [GO:0048856]; is part of pericardium development [GO:0060039]